{
  "gene_symbol": "SNW1",
  "term_label": "Unknown biological process",
  "gene_name": "SNW domain-containing protein 1",
  "term_id": "UNKNOWN:0002",
  "gene": "UniProtKB:Q13573"
}